T cell differentiation involved in immune response [GO:0002292] (biological process) Note: Note that immunologists typically use the word 'development' to refer to cells of B or T cell lineages undergoing the process that GO describes as 'cell differentiation'. Definition: The process in which an antigenically naive T cell acquires the specialized features of an effector, regulatory, or memory T cell as part of an immune response. Effector T cells include cells which provide T cell help or exhibit cytotoxicity towards other cells. Relationships: is a type of T cell activation involved in immune response [GO:0002286]; is a type of T cell differentiation [GO:0030217] Sources: GOC:add, ISBN:0781735149 Also known as: T cell development involved in immune response, T cell differentiation during immune response, T lymphocyte differentiation during immune response, T-cell differentiation during immune response, T-lymphocyte differentiation during immune response Subtypes: alpha-beta T cell differentiation involved in immune response [GO:0002293], GO:0002303, GO:0043379